{
  "gene_name": "Mortality factor 4-like protein 1",
  "gene": "UniProtKB:Q9UBU8",
  "term_label": "Unknown biological process",
  "gene_symbol": "MORF4L1",
  "term_id": "UNKNOWN:0002"
}